serous membrane development [GO:1904817] (biological process) Also known as: tunica serosa development, wall of serous sac development, serosa development Definition: The process whose specific outcome is the progression of a serous membrane over time, from its formation to the mature structure. References: PMID:15840053 Sources: GOC:TermGenie, GOC:dph, GO_REF:0000094 Relationships: is a type of anatomical structure development [GO:0048856] Subtypes: peritoneum development [GO:1904820]